left/right pattern formation [GO:0060972] (biological process) Definition: The pattern specification process that results in the subdivision of the left/right axis in space to define an area or volume in which specific patterns of cell differentiation will take place or in which cells interpret a specific environment. Sources: GOC:mtg_heart Relationships: is a type of regionalization [GO:0003002] Subtypes: embryonic heart tube left/right pattern formation [GO:0060971]